{
  "gene": "UniProtKB:Q5H9K5",
  "term_label": "Unknown molecular function",
  "gene_name": "Zinc finger matrin-type protein 1",
  "term_id": "UNKNOWN:0001",
  "gene_symbol": "ZMAT1"
}